{
  "term_label": "cytosolic ribosome assembly",
  "gene_symbol": "EFL1",
  "gene_name": "Elongation factor-like GTPase 1",
  "term_id": "GO:0042256",
  "gene": "UniProtKB:Q7Z2Z2"
}